specific granule membrane [GO:0035579] (cellular component) References: PMID:7334549 Sources: GOC:bf Also known as: secondary granule membrane Definition: The lipid bilayer surrounding a specific granule, a granule with a membranous, tubular internal structure, found primarily in mature neutrophil cells. Most are released into the extracellular fluid. Specific granules contain lactoferrin, lysozyme, vitamin B12 binding protein and elastase. Relationships: is a type of secretory granule membrane [GO:0030667]; is part of specific granule [GO:0042581]